{
  "term_label": "microtubule binding",
  "gene_name": "Centrosomal protein of 57 kDa",
  "gene": "UniProtKB:Q86XR8",
  "term_id": "GO:0008017",
  "gene_symbol": "CEP57"
}